{
  "term_id": "UNKNOWN:0002",
  "term_label": "Unknown biological process",
  "gene": "UniProtKB:A0A087WV53",
  "gene_symbol": "SPEGNB",
  "gene_name": "SPEG neighbor protein"
}